microspike [GO:0044393] (cellular component) References: PMID:11429692, PMID:12153987, PMID:19095735 Relationships: is a type of plasma membrane bounded cell projection [GO:0120025] Note: Although in some literature 'microspike' and 'filopodium' are used synonymously, in GO microspike refers to a cell projection that is distinct from a filopodium. See also 'filopodium ; GO:0030175'. Definition: A dynamic, actin-rich projection extending from the surface of a migrating animal cell.